{
  "gene_name": "Protein FAM9B",
  "gene": "UniProtKB:Q8IZU0",
  "gene_symbol": "FAM9B",
  "term_id": "GO:0051321",
  "term_label": "meiotic cell cycle"
}